{
  "term_label": "Unknown biological process",
  "term_id": "UNKNOWN:0002",
  "gene_name": "Annexin A3",
  "gene": "UniProtKB:P12429",
  "gene_symbol": "ANXA3"
}